regulation of response to cytokinesis checkpoint signaling [GO:1902147] (biological process) Relationships: is a type of regulation of response to cell cycle checkpoint signaling [GO:1902145]; regulates response to cytokinesis checkpoint signaling [GO:0072399] Also known as: regulation of cytokinesis checkpoint effector process, regulation of response to signal involved in cytokinesis checkpoint Subtypes: positive regulation of response to cytokinesis checkpoint signaling [GO:1902148] Sources: GOC:TermGenie, GOC:mtg_cell_cycle Definition: Any process that modulates the frequency, rate or extent of response to cytokinesis checkpoint signaling.